myoblast proliferation [GO:0051450] (biological process) Regulation: positively regulated by GO:2000288; RO_0002211 by regulation of myoblast proliferation [GO:2000291]; negatively regulated by negative regulation of myoblast proliferation [GO:2000818] Relationships: is a type of cell population proliferation [GO:0008283] Definition: The multiplication or reproduction of myoblasts, resulting in the expansion of a myoblast cell population. A myoblast is a mononucleate cell type that, by fusion with other myoblasts, gives rise to the myotubes that eventually develop into skeletal muscle fibers. Subtypes: myoblast proliferation involved in skeletal muscle regeneration [GO:0014844], cardiac muscle myoblast proliferation [GO:0110021] Sources: CL:0000056, GOC:ai, GOC:mtg_muscle